prospore membrane [GO:0005628] (cellular component) Sources: ISBN:0879693649 Relationships: is a type of GO:0016020; is part of ascospore-type prospore [GO:0042764] Definition: The prospore membrane is a double-membraned structure that extends from the cytoplasmic face of the spindle pole bodies to encompass the spindle pole bodies and the four nuclear lobes that are formed during meiosis. It helps isolate the meiotic nuclei from the cytoplasm during spore formation and serves as a foundation for the formation of the spore walls. An example of this component is found in Schizosaccharomyces pombe. Also known as: FSM, ascospore-type prospore membrane, forespore membrane